{
  "gene": "UniProtKB:P61018",
  "term_id": "GO:0005525",
  "term_label": "GTP binding",
  "gene_name": "Ras-related protein Rab-4B",
  "gene_symbol": "RAB4B"
}